{
  "term_id": "GO:0006024",
  "gene": "UniProtKB:Q96L58",
  "gene_symbol": "B3GALT6",
  "term_label": "glycosaminoglycan biosynthetic process",
  "gene_name": "Beta-1,3-galactosyltransferase 6"
}